metalloendopeptidase activity involved in amyloid precursor protein catabolic process [GO:1902945] (molecular function) Relationships: is a type of metalloendopeptidase activity [GO:0004222]; is part of GO:0042987 References: PMID:14598310, PMID:17855360 Sources: GOC:TermGenie, GOC:sjp, GO_REF:0000061 Definition: Any metalloendopeptidase activity that is involved in amyloid precursor protein catabolic process. Also known as: metalloendopeptidase activity involved in APP catabolic process, metalloendopeptidase activity involved in APP catabolism, metalloendopeptidase activity involved in amyloid precursor protein breakdown, metalloendopeptidase activity involved in amyloid precursor protein catabolism, metalloendopeptidase activity involved in amyloid precursor protein degradation, metalloendoprotease activity involved in APP catabolic process, metalloendoprotease activity involved in APP catabolism, metalloendoprotease activity involved in amyloid precursor protein breakdown, metalloendoprotease activity involved in amyloid precursor protein catabolic process, metalloendoprotease activity involved in amyloid precursor protein catabolism, metalloendoprotease activity involved in amyloid precursor protein degradation, metalloendoproteinase activity involved in APP catabolic process, metalloendoproteinase activity involved in APP catabolism, metalloendoproteinase activity involved in amyloid precursor protein breakdown, metalloendoproteinase activity involved in amyloid precursor protein catabolic process, metalloendoproteinase activity involved in amyloid precursor protein catabolism, metalloendoproteinase activity involved in amyloid precursor protein degradation